{
  "term_label": "regulation of systemic arterial blood pressure",
  "gene": "UniProtKB:P06870",
  "term_id": "GO:0003073",
  "gene_name": "Kallikrein-1",
  "gene_symbol": "KLK1"
}